{
  "gene_symbol": "RB1CC1",
  "term_id": "GO:0061723",
  "gene": "UniProtKB:Q8TDY2",
  "gene_name": "RB1-inducible coiled-coil protein 1",
  "term_label": "glycophagy"
}